{
  "term_id": "GO:0005886",
  "gene": "UniProtKB:Q9NS93",
  "gene_name": "Transmembrane 7 superfamily member 3",
  "gene_symbol": "TM7SF3",
  "term_label": "plasma membrane"
}